adenyl deoxyribonucleotide binding [GO:0032558] (molecular function) Relationships: is a type of adenyl nucleotide binding [GO:0030554]; is a type of purine deoxyribonucleotide binding [GO:0032554] Sources: GOC:mah Definition: Binding to an adenyl deoxyribonucleotide, any compound consisting of adenosine esterified with (ortho)phosphate or an oligophosphate at any hydroxyl group on the deoxyribose moiety. Subtypes: dAMP binding [GO:0032562], GO:0032563, dATP binding [GO:0032564]